epidermal stem cell homeostasis [GO:0036334] (biological process) Definition: Any biological process involved in the maintenance of the steady-state number of epidermal stem cells within a population of cells. References: PMID:17666529 Sources: CL:1000428, GOC:nhn Relationships: is a type of homeostasis of number of cells [GO:0048872]